{
  "term_label": "nucleoplasm",
  "gene_symbol": "ZNF641",
  "gene": "UniProtKB:Q96N77",
  "gene_name": "Zinc finger protein 641",
  "term_id": "GO:0005654"
}